positive regulation of telomere capping [GO:1904355] (biological process) Also known as: positive regulation of telomere end protection, up regulation of telomere capping, up regulation of telomere end protection, up-regulation of telomere capping, up-regulation of telomere end protection, upregulation of telomere capping, upregulation of telomere end protection, activation of telomere capping, activation of telomere end protection Definition: Any process that activates or increases the frequency, rate or extent of telomere capping. Relationships: is a type of positive regulation of telomere maintenance [GO:0032206]; is_a regulation of telomere capping [GO:1904353]; positively regulates GO:0016233 References: PMID:23959892 Sources: GOC:BHF, GOC:BHF_telomere, GOC:TermGenie, GOC:nc, GO_REF:0000058